negative regulation of metula development [GO:0070803] (biological process) Definition: Any process that stops, prevents, or reduces the frequency, rate or extent of metula development, a process that leads to the formation of metulae. Metulae are elongated mononucleate cells that bud from the surface of the conidiophore tip. Sources: GOC:mah Relationships: is a type of negative regulation of cell development [GO:0010721]; is a type of regulation of metula development [GO:0070802]; is a type of negative regulation of reproductive process [GO:2000242]; negatively regulates metula development [GO:0070789]